{
  "term_label": "enteric nervous system development",
  "gene_name": "Transcription factor SOX-8",
  "gene": "UniProtKB:P57073",
  "gene_symbol": "SOX8",
  "term_id": "GO:0048484"
}